{
  "term_id": "GO:0006094",
  "gene_symbol": "FBP1",
  "term_label": "gluconeogenesis",
  "gene_name": "Fructose-1,6-bisphosphatase 1",
  "gene": "UniProtKB:P09467"
}